{
  "term_label": "Unknown cellular component",
  "gene_symbol": "WAPL",
  "term_id": "UNKNOWN:0003",
  "gene": "UniProtKB:Q7Z5K2",
  "gene_name": "Wings apart-like protein homolog"
}